{
  "gene_name": "Platelet-derived growth factor D",
  "term_label": "platelet-derived growth factor receptor binding",
  "gene_symbol": "PDGFD",
  "term_id": "GO:0005161",
  "gene": "UniProtKB:Q9GZP0"
}